{
  "gene": "UniProtKB:P28328",
  "gene_symbol": "PEX2",
  "term_label": "peroxisome organization",
  "term_id": "GO:0007031",
  "gene_name": "Peroxisome biogenesis factor 2"
}